{
  "gene_name": "Transmembrane protein 255B",
  "gene": "UniProtKB:Q8WV15",
  "term_id": "UNKNOWN:0001",
  "term_label": "Unknown molecular function",
  "gene_symbol": "TMEM255B"
}